medulla oblongata development [GO:0021550] (biological process) Definition: The process whose specific outcome is the progression of the medulla oblongata over time, from its formation to the mature structure. The medulla oblongata lies directly above the spinal cord and controls vital autonomic functions such as digestion, breathing and the control of heart rate. Relationships: is a type of GO:0048856; BFO_0000050 hindbrain development [GO:0030902] Sources: GOC:cls, GOC:dgh, GOC:dph, GOC:jid, GO_REF:0000021 Also known as: medulla development, myelencephalon development